{
  "gene_name": "Myb-related protein B",
  "term_label": "positive regulation of transcription by RNA polymerase II",
  "gene_symbol": "MYBL2",
  "gene": "UniProtKB:P10244",
  "term_id": "GO:0045944"
}